{
  "term_label": "nucleus",
  "gene_name": "DNA replication licensing factor MCM5",
  "gene_symbol": "MCM5",
  "gene": "UniProtKB:P33992",
  "term_id": "GO:0005634"
}